{
  "gene_symbol": "AOC3",
  "gene_name": "Membrane primary amine oxidase",
  "term_id": "GO:0005507",
  "term_label": "copper ion binding",
  "gene": "UniProtKB:Q16853"
}